polytene chromosome weak point [GO:0005702] (cellular component) Definition: A region of the polytene chromosome where the diameter is considerably decreased, probably resulting from local differences in chromosome organization. Sources: GOC:bf, ISBN:0120649012 Also known as: constriction Relationships: is a type of cellular anatomical structure [GO:0110165]; is part of polytene chromosome [GO:0005700]